{
  "gene_name": "Thioredoxin-like protein 4B",
  "gene": "UniProtKB:Q9NX01",
  "term_label": "Unknown biological process",
  "term_id": "UNKNOWN:0002",
  "gene_symbol": "TXNL4B"
}